{
  "gene_name": "Charged multivesicular body protein 1b",
  "term_id": "UNKNOWN:0001",
  "term_label": "Unknown molecular function",
  "gene_symbol": "CHMP1B",
  "gene": "UniProtKB:Q7LBR1"
}